{
  "term_id": "GO:0005829",
  "term_label": "cytosol",
  "gene_symbol": "PLIN5",
  "gene": "UniProtKB:Q00G26",
  "gene_name": "Perilipin-5"
}